{
  "gene": "UniProtKB:P54826",
  "term_id": "UNKNOWN:0001",
  "gene_symbol": "GAS1",
  "gene_name": "Growth arrest-specific protein 1",
  "term_label": "Unknown molecular function"
}